{
  "term_id": "GO:0060294",
  "term_label": "cilium movement involved in cell motility",
  "gene_name": "Dynein axonemal heavy chain 7",
  "gene": "UniProtKB:Q8WXX0",
  "gene_symbol": "DNAH7"
}